positive regulation of glutamate secretion [GO:0014049] (biological process) Also known as: up regulation of glutamate secretion, up-regulation of glutamate secretion, upregulation of glutamate secretion, activation of glutamate secretion, stimulation of glutamate secretion Definition: Any process that activates or increases the frequency, rate or extent of the controlled release of glutamate. Subtypes: positive regulation of glutamate secretion, neurotransmission [GO:1903296] Relationships: is a type of GO:0014048; is a type of GO:0032892; is_a GO:0051957; is a type of GO:1903532; positively regulates GO:0014047 Sources: GOC:ef